{
  "gene_name": "CXXC-type zinc finger protein 5",
  "term_label": "methyl-CpG binding",
  "term_id": "GO:0008327",
  "gene_symbol": "CXXC5",
  "gene": "UniProtKB:Q7LFL8"
}